methylmalonate-semialdehyde dehydrogenase (acylating, NAD) activity [GO:0004491] (molecular function) Also known as: MMSA dehydrogenase activity, MSDH activity, methylmalonate-semialdehyde dehydrogenase (acylating) activity Definition: Catalysis of the reaction: 2-methyl-3-oxopropanoate + CoA + NAD+ = propanoyl-CoA + CO2 + NADH + H+. Can also use malonate (3-oxopropanoate) as a substrate. The reaction occurs in two steps with the decarboxylation process preceding CoA-binding. Bicarbonate rather than CO2 is released as a final product. References: PMID:2768248 Sources: EC:1.2.1.27 Relationships: is a type of oxidoreductase activity, acting on the aldehyde or oxo group of donors, NAD or NADP as acceptor [GO:0016620]